{
  "gene_name": "All trans-polyprenyl-diphosphate synthase PDSS2",
  "gene_symbol": "PDSS2",
  "term_id": "GO:0006744",
  "term_label": "ubiquinone biosynthetic process",
  "gene": "UniProtKB:Q86YH6"
}